cellular response to prostaglandin stimulus [GO:0071379] (biological process) Relationships: is a type of cellular response to hormone stimulus [GO:0032870]; is_a response to prostaglandin [GO:0034694]; is a type of cellular response to lipid [GO:0071396] Sources: GOC:mah Subtypes: cellular response to prostaglandin E stimulus [GO:0071380], cellular response to prostaglandin F stimulus [GO:0071381], GO:0071382, cellular response to prostaglandin D stimulus [GO:0071799] Definition: Any process that results in a change in state or activity of a cell (in terms of movement, secretion, enzyme production, gene expression, etc.) as a result of a prostagladin stimulus.